{
  "gene_name": "Plasminogen activator inhibitor 1",
  "gene": "UniProtKB:P05121",
  "term_label": "positive regulation of coagulation",
  "term_id": "GO:0050820",
  "gene_symbol": "SERPINE1"
}